regulation of gene expression [GO:0010468] (biological process) Note: This class covers any process that regulates the rate of production of a mature gene product, and so includes processes that regulate that rate by regulating the level, stability or availability of intermediates in the process of gene expression. For example, it covers any process that regulates the level, stability or availability of mRNA or circRNA for translation and thereby regulates the rate of production of the encoded protein via translation. Sources: GOC:txnOH-2018 Subtypes: regulation of cytokine production [GO:0001817], GO:0002331, regulation of production of molecular mediator of immune response [GO:0002700], regulation of DNA-templated transcription [GO:0006355], post-transcriptional regulation of gene expression [GO:0010608], GO:0010628, negative regulation of gene expression [GO:0010629], regulation of heterochromatin formation [GO:0031445], circadian regulation of gene expression [GO:0032922], epigenetic regulation of gene expression [GO:0040029], regulation of RNA splicing [GO:0043484], regulation of post-transcriptional gene silencing [GO:0060147], regulation of gene silencing by regulatory ncRNA [GO:0060966], regulation of mRNA catabolic process [GO:0061013], regulation of mitochondrial gene expression [GO:0062125], regulation of oxytocin production [GO:0140667], maternal-to-zygotic transition of gene expression [GO:0160021], negative regulation of transcription initiation-coupled chromatin remodeling [GO:0160217], GO:1902796, regulation of protein maturation [GO:1903317], regulation of rRNA processing [GO:2000232], regulation of tRNA processing [GO:2000235] Definition: Any process that modulates the frequency, rate or extent of gene expression. Gene expression is the process in which a gene's coding sequence is converted into a mature gene product (protein or RNA). Relationships: is a type of regulation of macromolecule biosynthetic process [GO:0010556]; regulates gene expression [GO:0010467] Also known as: regulation of protein expression, gene regulation, regulation of gene product expression